{
  "gene_symbol": "RDH13",
  "gene_name": "Retinol dehydrogenase 13",
  "term_id": "GO:0042574",
  "gene": "UniProtKB:Q8NBN7",
  "term_label": "retinal metabolic process"
}